{
  "gene": "UniProtKB:Q8NGI4",
  "term_label": "plasma membrane",
  "term_id": "GO:0005886",
  "gene_symbol": "OR4D11",
  "gene_name": "Olfactory receptor 4D11"
}